B cell chemotaxis across high endothelial venule [GO:0035769] (biological process) Definition: The movement of a B cell to cross a high endothelial venule in response to an external stimulus. Relationships: is a type of GO:0002518; is a type of GO:0035754 Sources: CL:0000236, GOC:BHF Also known as: B-cell chemotaxis across high endothelial venule